defense response to Gram-negative bacterium [GO:0050829] (biological process) Definition: Reactions triggered in response to the presence of a Gram-negative bacterium that act to protect the cell or organism. Relationships: is a type of defense response to bacterium [GO:0042742] Sources: GOC:ai Also known as: defence response to Gram-negative bacteria, defence response to Gram-negative bacterium, defense response to Gram-negative bacteria, Gram-negative antibacterial peptide activity